{
  "gene_symbol": "TTMP",
  "term_id": "UNKNOWN:0003",
  "gene_name": "TPA-induced transmembrane protein",
  "term_label": "Unknown cellular component",
  "gene": "UniProtKB:Q5BVD1"
}